{
  "gene": "UniProtKB:Q9Y468",
  "term_id": "GO:0042393",
  "gene_symbol": "L3MBTL1",
  "term_label": "histone binding",
  "gene_name": "Lethal(3)malignant brain tumor-like protein 1"
}